{
  "gene": "UniProtKB:Q9H4A5",
  "term_label": "cytosol",
  "gene_name": "Golgi phosphoprotein 3-like",
  "term_id": "GO:0005829",
  "gene_symbol": "GOLPH3L"
}